{
  "gene_symbol": "CSTPP1",
  "term_id": "UNKNOWN:0003",
  "gene_name": "Centriolar satellite-associated tubulin polyglutamylase complex regulator 1",
  "gene": "UniProtKB:Q9H6J7",
  "term_label": "Unknown cellular component"
}